{
  "gene": "UniProtKB:Q96SU4",
  "gene_symbol": "OSBPL9",
  "term_label": "sterol binding",
  "term_id": "GO:0032934",
  "gene_name": "Oxysterol-binding protein-related protein 9"
}